nitric oxide-cGMP-mediated signaling [GO:0038060] (biological process) Relationships: is a type of nitric oxide mediated signal transduction [GO:0007263] Definition: An intracellular signaling cassette in which the signal is passed on within the cell by nitric oxide (NO) activating soluble guanylyl cyclase (sGC). Includes synthesis of nitric oxide, guanylyl cyclase activity, and downstream effectors that further transmit the signal within the cell following activation by cGMP. Also known as: NO-cGMP signaling pathway, canonical nitric oxide signaling, classical nitric oxide signaling, nitric oxide-cGMP-mediated signal transduction, nitric oxide-cGMP-mediated signaling pathway, nitric oxide-cGMP-mediated signalling pathway References: PMID:21549190, PMID:22019632 Sources: GOC:signaling Regulation: RO_0002211 by regulation of nitric oxide-cGMP mediated signal transduction [GO:0141149]; positively regulated by positive regulation of nitric oxide-cGMP mediated signal transduction [GO:0141150]; negatively regulated by GO:0141151